{
  "gene_name": "Polypeptide N-acetylgalactosaminyltransferase 2",
  "term_label": "Golgi apparatus",
  "gene": "UniProtKB:Q10471",
  "term_id": "GO:0005794",
  "gene_symbol": "GALNT2"
}